{
  "term_label": "membrane",
  "gene_symbol": "VPS51",
  "term_id": "GO:0016020",
  "gene": "UniProtKB:Q9UID3",
  "gene_name": "Vacuolar protein sorting-associated protein 51 homolog"
}